viral budding from inner nuclear membrane [GO:0046771] (biological process) Relationships: is a type of GO:0046765 Definition: The envelopment of a virus, in which the nucleocapsid evaginates from the host inner nuclear membrane system into the perinuclear space, thus acquiring a membrane envelope. Sources: ISBN:0072370319 Also known as: virus budding from inner nuclear membrane by viral capsid envelopment, inner nuclear membrane viral budding during viral capsid envelopment, viral budding from inner nuclear membrane by viral capsid envelopment, viral budding from inner nuclear membrane during viral capsid envelopment, virus budding from inner nuclear membrane during viral capsid envelopment